{
  "gene": "UniProtKB:Q07108",
  "gene_name": "Early activation antigen CD69",
  "gene_symbol": "CD69",
  "term_id": "UNKNOWN:0001",
  "term_label": "Unknown molecular function"
}